{
  "gene_name": "Synaptic vesicle glycoprotein 2A",
  "term_id": "UNKNOWN:0001",
  "gene_symbol": "SV2A",
  "term_label": "Unknown molecular function",
  "gene": "UniProtKB:Q7L0J3"
}